positive regulation of bile acid secretion [GO:0120189] (biological process) References: PMID:22767443 Sources: GOC:BHF, GOC:BHF_miRNA, GOC:rph Relationships: is a type of positive regulation of organic acid transport [GO:0032892]; is a type of positive regulation of secretion [GO:0051047]; is a type of GO:0120188; positively regulates bile acid secretion [GO:0032782] Definition: Any process that activates or increases the frequency, rate or extent of the controlled release of bile acid from a cell or a tissue.